{
  "gene": "UniProtKB:Q6DN72",
  "gene_symbol": "FCRL6",
  "gene_name": "Fc receptor-like protein 6",
  "term_id": "GO:0004888",
  "term_label": "transmembrane signaling receptor activity"
}